{
  "gene": "UniProtKB:Q9BZL6",
  "gene_symbol": "PRKD2",
  "term_label": "cytosol",
  "term_id": "GO:0005829",
  "gene_name": "Serine_threonine-protein kinase D2"
}